{
  "term_label": "3'-5' exonuclease activity",
  "gene_symbol": "EXD2",
  "term_id": "GO:0008408",
  "gene_name": "Exonuclease 3'-5' domain-containing protein 2",
  "gene": "UniProtKB:Q9NVH0"
}